{
  "gene": "UniProtKB:Q9Y2W2",
  "term_label": "Unknown cellular component",
  "gene_name": "WW domain-binding protein 11",
  "term_id": "UNKNOWN:0003",
  "gene_symbol": "WBP11"
}